regulation of octopamine signaling pathway involved in response to food [GO:2000139] (biological process) Subtypes: negative regulation of octopamine signaling pathway involved in response to food [GO:2000140], positive regulation of octopamine signaling pathway involved in response to food [GO:2000141] Also known as: regulation of octopamine signalling pathway involved in response to food Definition: Any process that modulates the frequency, rate or extent of octopamine signaling pathway involved in response to food. References: PMID:19609300 Sources: GOC:mah Relationships: is a type of regulation of octopamine signaling pathway [GO:2000128]; RO_0002211 octopamine signaling pathway involved in response to food [GO:0071935]